chloroplast inner membrane [GO:0009706] (cellular component) Sources: GOC:tb Definition: The inner, i.e. lumen-facing, lipid bilayer of the chloroplast envelope; also faces the chloroplast stroma. Relationships: is a type of plastid inner membrane [GO:0009528]; is a type of GO:0031969 Also known as: chloroplast inner envelope